regulation of lateral root development [GO:2000023] (biological process) Relationships: is_a regulation of post-embryonic root development [GO:2000069]; RO_0002211 lateral root development [GO:0048527] Sources: GOC:obol Definition: Any process that modulates the frequency, rate or extent of lateral root development. Subtypes: negative regulation of lateral root development [GO:1901332], positive regulation of lateral root development [GO:1901333]